{
  "gene_name": "Speckle-type POZ protein-like",
  "term_label": "proteasome-mediated ubiquitin-dependent protein catabolic process",
  "term_id": "GO:0043161",
  "gene_symbol": "SPOPL",
  "gene": "UniProtKB:Q6IQ16"
}